{
  "gene_name": "Ufm1-specific protease 2",
  "gene_symbol": "UFSP2",
  "term_id": "GO:0006508",
  "gene": "UniProtKB:Q9NUQ7",
  "term_label": "proteolysis"
}